cerebral cortex GABAergic interneuron development [GO:0021894] (biological process) Relationships: is a type of forebrain neuron development [GO:0021884]; is part of cerebral cortex GABAergic interneuron differentiation [GO:0021892] References: PMID:12626695 Sources: GOC:cls, GOC:dgh, GOC:dph, GOC:jid, GO_REF:0000021 Definition: The process whose specific outcome is the progression of a cerebral cortex GABAergic interneuron over time, from initial commitment to its fate, to the fully functional differentiated cell.